{
  "term_id": "GO:0005251",
  "term_label": "delayed rectifier potassium channel activity",
  "gene": "UniProtKB:O95259",
  "gene_symbol": "KCNH1",
  "gene_name": "Potassium voltage-gated channel subfamily H member 1"
}